{
  "term_label": "RNA polymerase II cis-regulatory region sequence-specific DNA binding",
  "gene": "UniProtKB:Q3KNS6",
  "gene_symbol": "ZNF829",
  "term_id": "GO:0000978",
  "gene_name": "Zinc finger protein 829"
}